{
  "gene": "UniProtKB:Q86Y56",
  "term_id": "GO:0005737",
  "gene_symbol": "DNAAF5",
  "gene_name": "Dynein axonemal assembly factor 5",
  "term_label": "cytoplasm"
}